{
  "gene": "UniProtKB:Q2UY09",
  "term_id": "GO:0031012",
  "gene_name": "Collagen alpha-1(XXVIII) chain",
  "term_label": "extracellular matrix",
  "gene_symbol": "COL28A1"
}